{
  "gene": "UniProtKB:Q96EP9",
  "gene_symbol": "SLC10A4",
  "term_id": "UNKNOWN:0003",
  "term_label": "Unknown cellular component",
  "gene_name": "Sodium_bile acid cotransporter 4"
}